positive regulation of macrophage differentiation [GO:0045651] (biological process) Relationships: is a type of positive regulation of myeloid leukocyte differentiation [GO:0002763]; is a type of regulation of macrophage differentiation [GO:0045649]; positively regulates macrophage differentiation [GO:0030225] Definition: Any process that activates or increases the frequency, rate or extent of macrophage differentiation. Sources: GOC:go_curators Also known as: up regulation of macrophage differentiation, up-regulation of macrophage differentiation, upregulation of macrophage differentiation, activation of macrophage differentiation, stimulation of macrophage differentiation Subtypes: positive regulation of microglia differentiation [GO:0014008]